{
  "gene_symbol": "ANKRD26P1",
  "term_id": "UNKNOWN:0001",
  "gene": "UniProtKB:Q6NSI1",
  "gene_name": "Putative ankyrin repeat domain-containing protein 26-like protein",
  "term_label": "Unknown molecular function"
}